{
  "gene": "UniProtKB:Q149N8",
  "gene_name": "E3 ubiquitin-protein ligase SHPRH",
  "term_label": "DNA damage response",
  "term_id": "GO:0006974",
  "gene_symbol": "SHPRH"
}